{
  "gene": "UniProtKB:Q9HCZ1",
  "gene_name": "Zinc finger protein 334",
  "term_label": "regulation of transcription by RNA polymerase II",
  "gene_symbol": "ZNF334",
  "term_id": "GO:0006357"
}